{
  "term_label": "P granule organization",
  "gene_name": "Tudor domain-containing protein 1",
  "gene": "UniProtKB:Q9BXT4",
  "term_id": "GO:0030719",
  "gene_symbol": "TDRD1"
}